{
  "gene_symbol": "MT-ND5",
  "gene": "UniProtKB:P03915",
  "term_id": "UNKNOWN:0001",
  "gene_name": "NADH-ubiquinone oxidoreductase chain 5",
  "term_label": "Unknown molecular function"
}